{
  "term_id": "GO:0005634",
  "term_label": "nucleus",
  "gene_name": "C-terminal-binding protein 1",
  "gene_symbol": "CTBP1",
  "gene": "UniProtKB:Q13363"
}